negative regulation of intrinsic apoptotic signaling pathway [GO:2001243] (BP) Definition: Any process that stops, prevents or reduces the frequency, rate or extent of intrinsic apoptotic signaling pathway. Relationships: is a type of GO:1902532; is a type of negative regulation of apoptotic signaling pathway [GO:2001234]; is a type of regulation of intrinsic apoptotic signaling pathway [GO:2001242]; negatively regulates intrinsic apoptotic signaling pathway [GO:0097193] Sources: GOC:mtg_apoptosis Also known as: negative regulation of intrinsic apoptotic pathway, negative regulation of intrinsic apoptotic signalling pathway, negative regulation of mitochondrial-mediated apoptotic pathway, negative regulation of intrinsic apoptosis Subtypes: negative regulation of oxidative stress-induced intrinsic apoptotic signaling pathway [GO:1902176], negative regulation of intrinsic apoptotic signaling pathway in response to osmotic stress [GO:1902219], negative regulation of intrinsic apoptotic signaling pathway in response to DNA damage [GO:1902230], negative regulation of endoplasmic reticulum stress-induced intrinsic apoptotic signaling pathway [GO:1902236], negative regulation of intrinsic apoptotic signaling pathway by p53 class mediator [GO:1902254], negative regulation of hypoxia-induced intrinsic apoptotic signaling pathway [GO:1903298], negative regulation of nitrosative stress-induced intrinsic apoptotic signaling pathway [GO:1905259]